regulation of interleukin-4 production [GO:0032673] (biological process) Definition: Any process that modulates the frequency, rate, or extent of interleukin-4 production. References: PMID:29778524 Sources: GOC:mah Also known as: regulation of IL-4 production, regulation of interleukin-4 biosynthetic process, regulation of interleukin-4 secretion Relationships: is a type of GO:0001817; RO_0002211 interleukin-4 production [GO:0032633] Subtypes: GO:0032713, positive regulation of interleukin-4 production [GO:0032753]